{
  "term_label": "ribosome",
  "term_id": "GO:0005840",
  "gene": "UniProtKB:P62266",
  "gene_symbol": "RPS23",
  "gene_name": "Small ribosomal subunit protein uS12"
}